{
  "term_label": "cysteine-type deubiquitinase activity",
  "gene_name": "Deubiquitinase OTUD6B",
  "term_id": "GO:0004843",
  "gene": "UniProtKB:Q8N6M0",
  "gene_symbol": "OTUD6B"
}